{
  "gene": "UniProtKB:Q9NWF9",
  "gene_name": "E3 ubiquitin-protein ligase RNF216",
  "gene_symbol": "RNF216",
  "term_id": "UNKNOWN:0003",
  "term_label": "Unknown cellular component"
}